{
  "gene_name": "Cyclin-dependent kinase 14",
  "term_id": "GO:0004693",
  "gene": "UniProtKB:O94921",
  "term_label": "cyclin-dependent protein serine/threonine kinase activity",
  "gene_symbol": "CDK14"
}